{
  "gene_symbol": "UNC119",
  "term_id": "GO:0045171",
  "term_label": "intercellular bridge",
  "gene_name": "Protein unc-119 homolog A",
  "gene": "UniProtKB:Q13432"
}